{
  "gene_name": "Keratin-associated protein 4-5",
  "gene_symbol": "KRTAP4-5",
  "term_id": "UNKNOWN:0001",
  "gene": "UniProtKB:Q9BYR2",
  "term_label": "Unknown molecular function"
}